bacterial-type flagellum stator complex [GO:0120101] (CC) Also known as: bacterial-type flagellum motor force generator complex, bacterial-type flagellum torque generator complex References: PMID:10572114, PMID:12624192, PMID:24697492, PMID:25251856 Sources: GOC:cilia Relationships: is a type of plasma membrane protein complex [GO:0098797]; is part of bacterial-type flagellum motor [GO:0120100] Definition: A hetero-hexameric complex of 2 membrane proteins, A and B, with stoichiometry A4B2. The A and B proteins form a channel through which flow the ions that power the bacterial-type flagellum. They form the stator, or nonrotating portion, of the flagellum motor with the B protein apparently attached to the peptidoglycan cell wall. Examples include the H+ driven MotA-MotB stator complex of Escherichia coli and Salmonella enterica, and the Na+ driven PomA-PomB stator complex of Vibrio and Shewanella species.